{
  "term_id": "GO:0005765",
  "gene": "UniProtKB:P01903",
  "term_label": "lysosomal membrane",
  "gene_symbol": "HLA-DRA",
  "gene_name": "HLA class II histocompatibility antigen, DR alpha chain"
}